mannose-1-phosphate guanylyltransferase (GTP) activity [GO:0004475] (molecular function) Sources: RHEA:15229 Also known as: mannose-1-phosphate guanylyltransferase activity, GTP:mannose-1-phosphate guanylyltransferase activity, GDP-mannose pyrophosphorylase activity, GTP-mannose-1-phosphate guanylyltransferase activity, GTP:alpha-D-mannose-1-phosphate guanylyltransferase activity, PIM-GMP (phosphomannose isomerase-guanosine 5'-diphospho-D-mannose pyrophosphorylase), guanosine 5'-diphospho-D-mannose pyrophosphorylase activity, guanosine diphosphomannose pyrophosphorylase activity, guanosine triphosphate-mannose 1-phosphate guanylyltransferase activity, mannose 1-phosphate guanylyltransferase (guanosine triphosphate) Definition: Catalysis of the reaction: alpha-D-mannose 1-phosphate + GTP = diphosphate + GDP-alpha-D-mannose. Relationships: is a type of guanylyltransferase activity [GO:0070568]